{
  "term_label": "regulation of cell population proliferation",
  "term_id": "GO:0042127",
  "gene_name": "Transcription factor AP-2-delta",
  "gene": "UniProtKB:Q7Z6R9",
  "gene_symbol": "TFAP2D"
}